leg disc pattern formation [GO:0035223] (biological process) Sources: GOC:bf Relationships: is a type of GO:0007447; is part of GO:0035218 Definition: The process that gives rise to the patterns of cell differentiation in the leg imaginal disc. Subtypes: leg disc proximal/distal pattern formation [GO:0007479], leg disc anterior/posterior pattern formation [GO:0035200]